{
  "gene": "UniProtKB:P0DN82",
  "term_id": "GO:0050911",
  "gene_symbol": "OR12D1",
  "term_label": "detection of chemical stimulus involved in sensory perception of smell",
  "gene_name": "Olfactory receptor 12D1"
}